{
  "term_label": "Unknown biological process",
  "term_id": "UNKNOWN:0002",
  "gene_name": "UPF0193 protein EVG1",
  "gene_symbol": "C22orf23",
  "gene": "UniProtKB:Q9BZE7"
}